{
  "term_label": "plasma membrane",
  "gene_symbol": "CLDN20",
  "gene": "UniProtKB:P56880",
  "term_id": "GO:0005886",
  "gene_name": "Claudin-20"
}